GTP-dependent protein kinase activity [GO:0034211] (molecular function) References: PMID:17200152 Sources: GOC:ecd Relationships: is a type of GO:0004674 Note: The reaction requires the presence of GTP. Definition: GTP dependent catalysis of the reaction: ATP + a protein serine/threonine = ADP + protein serine/threonine phosphate.